{
  "term_id": "GO:0005829",
  "gene_name": "Phosphoribosyltransferase domain-containing protein 1",
  "gene_symbol": "PRTFDC1",
  "gene": "UniProtKB:Q9NRG1",
  "term_label": "cytosol"
}